negative regulation of TORC1 signaling [GO:1904262] (biological process) References: PMID:25366275 Sources: GOC:TermGenie, GO_REF:0000058 Definition: Any process that stops, prevents or reduces the frequency, rate or extent of TORC1 signaling. Relationships: is a type of negative regulation of TOR signaling [GO:0032007]; is a type of GO:1903432; negatively regulates TORC1 signaling [GO:0038202] Also known as: down regulation of TORC1 signal transduction, down regulation of TORC1 signaling, down-regulation of TORC1 signal transduction, down-regulation of TORC1 signaling, downregulation of TORC1 signal transduction, downregulation of TORC1 signaling, negative regulation of TORC1 signal transduction, inhibition of TORC1 signal transduction, inhibition of TORC1 signaling